{
  "gene_symbol": "GALM",
  "term_id": "GO:0004034",
  "gene": "UniProtKB:Q96C23",
  "gene_name": "Galactose mutarotase",
  "term_label": "aldose 1-epimerase activity"
}